{
  "term_id": "GO:0046705",
  "gene_symbol": "CMPK1",
  "gene_name": "UMP-CMP kinase",
  "term_label": "CDP biosynthetic process",
  "gene": "UniProtKB:P30085"
}